{
  "gene_name": "Protein CUSTOS",
  "gene_symbol": "CUSTOS",
  "term_label": "Spemann organizer formation",
  "gene": "UniProtKB:Q96C57",
  "term_id": "GO:0060061"
}